{
  "term_label": "detection of bacterium",
  "gene": "UniProtKB:Q13075",
  "gene_name": "Baculoviral IAP repeat-containing protein 1",
  "term_id": "GO:0016045",
  "gene_symbol": "NAIP"
}